{
  "term_label": "keratohyalin granule",
  "gene_symbol": "HRNR",
  "gene_name": "Hornerin",
  "gene": "UniProtKB:Q86YZ3",
  "term_id": "GO:0036457"
}